{
  "gene_name": "F-box_WD repeat-containing protein 2",
  "term_label": "Unknown cellular component",
  "gene_symbol": "FBXW2",
  "gene": "UniProtKB:Q9UKT8",
  "term_id": "UNKNOWN:0003"
}